RNA replication [GO:0039703] (biological process) Relationships: is a type of GO:0016070; has part RNA biosynthetic process [GO:0032774] Definition: The cellular metabolic process in which a cell duplicates one or more molecules of RNA. Sources: GOC:bf, GOC:jl